rhamnogalacturonan II biosynthetic process [GO:0010306] (biological process) Relationships: is a type of cell wall pectin biosynthetic process [GO:0052325] References: PMID:12754267 Definition: The chemical reactions and pathways resulting in the formation of rhamnogalacturonan II, a low molecular mass (5 - 10KDa) pectic polysaccharide, conserved in the primary walls of dicotyledenous and monocotyledenous plants and gymnosperms.